stromal side of plastid inner membrane [GO:0098570] (cellular component) Definition: The side (leaflet) of the plastid inner membrane that faces the stroma, and any proteins embedded in it or loosely bound to its surface. Sources: GOC:dos Relationships: is a type of GO:0098552; is part of GO:0009528